premeiotic DNA replication preinitiation complex assembly [GO:1902976] (biological process) Sources: GOC:TermGenie, GO_REF:0000060 Definition: Any DNA replication preinitiation complex assembly that is involved in meiotic cell cycle. Also known as: DNA replication preinitiation complex formation involved in meiotic cell cycle, pre-IC complex assembly involved in meiotic cell cycle Relationships: is a type of DNA replication preinitiation complex assembly [GO:0071163]; is a type of meiotic cell cycle process [GO:1903046]; is part of premeiotic DNA replication [GO:0006279]